{
  "term_id": "GO:0042073",
  "gene_name": "Intraflagellar transport protein 27 homolog",
  "gene": "UniProtKB:Q9BW83",
  "term_label": "intraciliary transport",
  "gene_symbol": "IFT27"
}